meiotic spindle formation (spindle phase two) [GO:0140642] (biological process) Definition: The spindle organization process in which the spindle is maintained at a constant length during meiotic metaphase. References: PMID:32723864 Relationships: is a type of GO:0090306